{
  "gene": "UniProtKB:O95867",
  "gene_symbol": "LY6G6C",
  "term_label": "Unknown biological process",
  "gene_name": "Lymphocyte antigen 6 complex locus protein G6c",
  "term_id": "UNKNOWN:0002"
}